heterochromatin-nuclear membrane anchor activity [GO:0062239] (molecular function) Definition: Binding to heterochromatin and the nuclear inner membrane, in order to establish and maintain the heterochromatin location and organization. References: PMID:31635174 Also known as: heterochromatin-nuclear membrane tether activity, nuclear membrane-heterochromatin anchor activity, nuclear membrane-heterochromatin tether activity Relationships: is a type of chromatin-nuclear membrane anchor activity [GO:0140707]